pentasaccharide transport [GO:2001100] (biological process) Regulation: regulated by GO:1900360; negatively regulated by negative regulation of pentasaccharide transport [GO:1900361]; positively regulated by GO:1900362 Definition: The directed movement of a pentasaccharideacetate into, out of or within a cell, or between cells, by means of some agent such as a transporter or pore. Subtypes: GO:2001101 Relationships: is a type of oligosaccharide transport [GO:0015772] Sources: GOC:mengo_curators